{
  "gene_symbol": "KRT6B",
  "gene": "UniProtKB:P04259",
  "term_id": "GO:0030280",
  "gene_name": "Keratin, type II cytoskeletal 6B",
  "term_label": "structural constituent of skin epidermis"
}